spermine transmembrane transport [GO:1903710] (biological process) References: PMID:15637075 Sources: GOC:TermGenie, GO_REF:0000069 Relationships: is_a spermine transport [GO:0000296]; is a type of polyamine transmembrane transport [GO:1902047] Definition: The process in which spermine is transported across a membrane.